{
  "gene_name": "Growth arrest-specific protein 6",
  "gene": "UniProtKB:Q14393",
  "term_label": "extracellular space",
  "term_id": "GO:0005615",
  "gene_symbol": "GAS6"
}